{
  "term_label": "mitochondrion",
  "gene_name": "Large ribosomal subunit protein mL39",
  "gene_symbol": "MRPL39",
  "gene": "UniProtKB:Q9NYK5",
  "term_id": "GO:0005739"
}